cellular response to amino acid stimulus [GO:0071230] (biological process) Definition: Any process that results in a change in state or activity of a cell (in terms of movement, secretion, enzyme production, gene expression, etc.) as a result of an amino acid stimulus. An amino acid is a carboxylic acids containing one or more amino groups. Sources: GOC:mah Also known as: cellular response to amino acid Relationships: is a type of response to amino acid [GO:0043200]; is a type of GO:0071229 Subtypes: cellular response to L-canavanine [GO:0036280], cellular response to L-cysteine [GO:0036346], cellular response to methionine [GO:0061431], cellular response to 1-aminocyclopropane-1-carboxylic acid [GO:0071213], cellular response to histidine [GO:0071232], cellular response to L-leucine [GO:0071233], cellular response to phenylalanine [GO:0071234], cellular response to proline [GO:0071235], cellular response to L-thialysine [GO:0072751], cellular response to thyroxine stimulus [GO:0097069], cellular response to L-arginine [GO:1903577], cellular response to kainic acid [GO:1904374], cellular response to L-dopa [GO:1904474], GO:1904845, cellular response to L-glutamate [GO:1905232], cellular response to 3,3',5-triiodo-L-thyronine [GO:1905243], cellular response to homocysteine [GO:1905375], cellular response to glycine [GO:1905430]